{
  "gene_name": "Rho-related BTB domain-containing protein 2",
  "term_label": "cortical cytoskeleton organization",
  "gene": "UniProtKB:Q9BYZ6",
  "gene_symbol": "RHOBTB2",
  "term_id": "GO:0030865"
}